{
  "term_label": "Unknown biological process",
  "gene_name": "Protein FAM185A",
  "gene": "UniProtKB:Q8N0U4",
  "gene_symbol": "FAM185A",
  "term_id": "UNKNOWN:0002"
}